{
  "term_label": "release of sequestered calcium ion into cytosol",
  "gene_name": "1-phosphatidylinositol 4,5-bisphosphate phosphodiesterase gamma-1",
  "gene": "UniProtKB:P19174",
  "gene_symbol": "PLCG1",
  "term_id": "GO:0051209"
}